{
  "gene_name": "Protein phosphatase Slingshot homolog 1",
  "term_id": "GO:0004721",
  "gene": "UniProtKB:Q8WYL5",
  "gene_symbol": "SSH1",
  "term_label": "phosphoprotein phosphatase activity"
}